{
  "term_id": "GO:0005739",
  "gene_symbol": "HTATIP2",
  "gene_name": "Oxidoreductase HTATIP2",
  "term_label": "mitochondrion",
  "gene": "UniProtKB:Q9BUP3"
}